indoleacetate-lysine synthetase activity [GO:0047721] (molecular function) Sources: EC:6.3.2.20, RHEA:14857 Definition: Catalysis of the reaction: (indol-3-yl)acetate + L-lysine + ATP = N(6)-[(indole-3-yl)acetyl]-L-lysine + ADP + 2 H+ + phosphate. Relationships: is a type of indole-3-acetic acid amido synthetase activity [GO:0010279] Also known as: indoleacetate-lysine ligase activity, (indol-3-yl)acetate:L-lysine ligase (ADP-forming), IAA-lysine synthetase activity, N-(indole-3-acetyl)-L-lysine synthetase activity, indoleacetate:L-lysine ligase (ADP-forming)